induction of bacterial agglutination [GO:0043152] (biological process) Relationships: is a type of GO:0019731 Definition: Any process in which infecting bacteria are clumped together by a host organism. Sources: GOC:jl